{
  "term_id": "GO:0005789",
  "gene_symbol": "ITPR2",
  "term_label": "endoplasmic reticulum membrane",
  "gene_name": "Inositol 1,4,5-trisphosphate receptor type 2",
  "gene": "UniProtKB:Q14571"
}